positive regulation of integrin activation by cell surface receptor linked signal transduction [GO:0033626] (BP) Also known as: cell surface receptor linked signal transduction leading to integrin activation, cell surface receptor linked signal transduction leading to integrin complex activation References: PMID:12213832, PMID:14754902 Sources: GOC:add Definition: Any process that activates or increases the frequency, rate, or extent of integrin activation by cell surface receptor linked signal transduction. This can occur by increased affinity of an integrin for its extracellular ligands. Relationships: is a type of GO:0007166; is a type of positive regulation of integrin activation [GO:0033625]